{
  "gene_symbol": "PHKA1",
  "term_label": "Unknown molecular function",
  "term_id": "UNKNOWN:0001",
  "gene_name": "Phosphorylase b kinase regulatory subunit alpha, skeletal muscle isoform",
  "gene": "UniProtKB:P46020"
}